{
  "gene_name": "Protein FAM131C",
  "gene": "UniProtKB:Q96AQ9",
  "term_id": "UNKNOWN:0002",
  "gene_symbol": "FAM131C",
  "term_label": "Unknown biological process"
}